{
  "gene_symbol": "ST13P4",
  "gene": "UniProtKB:Q8IZP2",
  "gene_name": "Putative protein FAM10A4",
  "term_id": "UNKNOWN:0001",
  "term_label": "Unknown molecular function"
}